{
  "gene": "UniProtKB:P25100",
  "term_id": "GO:0004937",
  "gene_name": "Alpha-1D adrenergic receptor",
  "term_label": "alpha1-adrenergic receptor activity",
  "gene_symbol": "ADRA1D"
}